{
  "term_label": "dendrite",
  "gene": "UniProtKB:Q86UL8",
  "gene_symbol": "MAGI2",
  "term_id": "GO:0030425",
  "gene_name": "Membrane-associated guanylate kinase, WW and PDZ domain-containing protein 2"
}